ruffle assembly [GO:0097178] (biological process) Also known as: membrane ruffle formation, membrane ruffling Relationships: is a type of GO:0031529; is a type of plasma membrane bounded cell projection assembly [GO:0120031] Definition: The aggregation, arrangement and bonding together of a set of components to form a ruffle, a projection at the leading edge of a crawling cell; the protrusions are supported by a microfilament meshwork. The formation of ruffles (also called membrane ruffling) is thought to be controlled by a group of enzymes known as Rho GTPases, specifically RhoA, Rac1 and cdc42. Regulation: regulated by regulation of ruffle assembly [GO:1900027]; negatively regulated by GO:1900028; positively regulated by positive regulation of ruffle assembly [GO:1900029] References: PMID:12556481 Sources: GOC:yaf, Wikipedia:Membrane_ruffling